positive regulation of sclerenchyma cell differentiation [GO:1904369] (BP) References: PMID:26025534 Sources: GOC:TermGenie, GO_REF:0000058 Definition: Any process that activates or increases the frequency, rate or extent of sclerenchyma cell differentiation. Also known as: up regulation of sclerenchyma cell differentiation, up-regulation of sclerenchyma cell differentiation, upregulation of sclerenchyma cell differentiation Relationships: is a type of GO:0045597; is a type of regulation of sclerenchyma cell differentiation [GO:1904368]; positively regulates sclerenchyma cell differentiation [GO:0014001]